{
  "gene_name": "Dystroglycan 1",
  "gene": "UniProtKB:Q14118",
  "gene_symbol": "DAG1",
  "term_label": "extracellular space",
  "term_id": "GO:0005615"
}